taurine transmembrane transport [GO:0015734] (biological process) Sources: GOC:krc Also known as: taurine transport Relationships: is a type of alkanesulfonate transmembrane transport [GO:0042918]; is a type of nitrogen compound transport [GO:0071705] Definition: The directed movement of taurine into, out of or within a cell, or between cells, by means of some agent such as a transporter or pore.